{
  "gene": "UniProtKB:Q7Z5L7",
  "term_id": "UNKNOWN:0001",
  "gene_name": "Podocan",
  "gene_symbol": "PODN",
  "term_label": "Unknown molecular function"
}